{
  "gene_symbol": "TGFB1",
  "term_label": "extracellular space",
  "gene": "UniProtKB:P01137",
  "term_id": "GO:0005615",
  "gene_name": "Transforming growth factor beta-1 proprotein"
}